negative regulation of oxidative stress-induced intrinsic apoptotic signaling pathway [GO:1902176] (biological process) Definition: Any process that stops, prevents or reduces the frequency, rate or extent of an oxidative stress-induced intrinsic apoptotic signaling pathway. References: PMID:11672522 Sources: GOC:BHF, GOC:TermGenie, GOC:mtg_apoptosis Also known as: down regulation of intrinsic apoptotic signaling pathway in response to oxidative stress, down-regulation of intrinsic apoptotic signaling pathway in response to oxidative stress, downregulation of intrinsic apoptotic signaling pathway in response to oxidative stress, negative regulation of intrinsic apoptotic signaling pathway in response to oxidative stress, inhibition of intrinsic apoptotic signaling pathway in response to oxidative stress Relationships: is_a regulation of oxidative stress-induced intrinsic apoptotic signaling pathway [GO:1902175]; is a type of negative regulation of intrinsic apoptotic signaling pathway [GO:2001243]; RO_0002212 intrinsic apoptotic signaling pathway in response to oxidative stress [GO:0008631] Subtypes: negative regulation of oxidative stress-induced neuron intrinsic apoptotic signaling pathway [GO:1903377], negative regulation of intrinsic apoptotic signaling pathway in response to hydrogen peroxide [GO:1903751]